{
  "term_label": "extracellular space",
  "gene_name": "Membrane cofactor protein",
  "gene_symbol": "CD46",
  "term_id": "GO:0005615",
  "gene": "UniProtKB:P15529"
}